{
  "gene_symbol": "ZNF75A",
  "term_id": "GO:0005634",
  "term_label": "nucleus",
  "gene_name": "Zinc finger protein 75A",
  "gene": "UniProtKB:Q96N20"
}